{
  "gene_name": "Methyl-CpG-binding domain protein 3-like 1",
  "gene": "UniProtKB:Q8WWY6",
  "term_id": "GO:0005634",
  "gene_symbol": "MBD3L1",
  "term_label": "nucleus"
}